{
  "gene_symbol": "CDK5RAP1",
  "gene_name": "Mitochondrial tRNA methylthiotransferase CDK5RAP1",
  "gene": "UniProtKB:Q96SZ6",
  "term_id": "GO:0035597",
  "term_label": "tRNA-2-methylthio-N(6)-dimethylallyladenosine(37) synthase activity"
}